{
  "gene": "UniProtKB:Q8TEB1",
  "gene_symbol": "DCAF11",
  "term_label": "Cul4-RING E3 ubiquitin ligase complex",
  "gene_name": "DDB1- and CUL4-associated factor 11",
  "term_id": "GO:0080008"
}